{
  "gene": "UniProtKB:Q6UX71",
  "gene_name": "Plexin domain-containing protein 2",
  "gene_symbol": "PLXDC2",
  "term_id": "UNKNOWN:0002",
  "term_label": "Unknown biological process"
}